leghemoglobin reductase [NAD(P)H] activity [GO:0015043] (molecular function) Definition: Catalysis of the reaction: 2 Fe(III)-[leghemoglobin] + NAD(P)H = 2 Fe(II)-[leghemoglobin] + NAD(P)+ + H+. Also known as: leghemoglobin reductase activity, NAD(P)H:ferrileghemoglobin oxidoreductase activity, ferric leghemoglobin reductase activity Relationships: is_a oxidoreductase activity, acting on NAD(P)H, heme protein as acceptor [GO:0016653] Sources: EC:1.6.2.6